{
  "gene_name": "Sex comb on midleg-like protein 2",
  "gene": "UniProtKB:Q9UQR0",
  "term_id": "GO:0042393",
  "gene_symbol": "SCML2",
  "term_label": "histone binding"
}